{
  "gene_name": "Sphingosine-1-phosphate transporter SPNS2",
  "gene_symbol": "SPNS2",
  "term_label": "sphingosine-1-phosphate receptor signaling pathway",
  "gene": "UniProtKB:Q8IVW8",
  "term_id": "GO:0003376"
}